{
  "gene_name": "Hsp90 co-chaperone Cdc37",
  "term_id": "GO:0051082",
  "gene": "UniProtKB:Q16543",
  "term_label": "unfolded protein binding",
  "gene_symbol": "CDC37"
}